{
  "gene": "UniProtKB:O14713",
  "term_label": "cell periphery",
  "term_id": "GO:0071944",
  "gene_symbol": "ITGB1BP1",
  "gene_name": "Integrin beta-1-binding protein 1"
}